[Ni-Fe] hydrogenase complex [GO:0044569] (cellular component) References: PMID:8936309 Sources: GOC:mengo_curators, GOC:tt Definition: A microbial enzyme complex which contains nickel and iron in its active site. In Acetomicrobium flavidum it is an alpha 2 beta 2 tetramer. Also known as: Ni-Fe hydrogenase complex, nickel-iron hydrogenase complex Relationships: is_a catalytic complex [GO:1902494]